virus baseplate assembly [GO:0098045] (biological process) Definition: The aggregation, arrangement and bonding together of a set of components to form a virus baseplate. Sources: GOC:bm Relationships: is a type of GO:0016032; is part of viral tail assembly [GO:0098003]